imaginal disc-derived female genitalia morphogenesis [GO:0048804] (biological process) Also known as: female genital morphogenesis Sources: GOC:ai, GOC:sensu Definition: The process in which the anatomical structures of female genitalia are generated and organized from the genital disc. Relationships: is a type of GO:0048805; is_a GO:0048807; is part of imaginal disc-derived female genitalia development [GO:0007486]